{
  "term_label": "electron-transferring-flavoprotein dehydrogenase activity",
  "gene": "UniProtKB:Q9BRQ8",
  "gene_symbol": "AIFM2",
  "gene_name": "Ferroptosis suppressor protein 1",
  "term_id": "GO:0004174"
}